{
  "gene": "UniProtKB:A8MXZ3",
  "term_label": "Unknown biological process",
  "gene_name": "Keratin-associated protein 9-1",
  "gene_symbol": "KRTAP9-1",
  "term_id": "UNKNOWN:0002"
}